{
  "gene_symbol": "SETD4",
  "gene": "UniProtKB:Q9NVD3",
  "gene_name": "SET domain-containing protein 4",
  "term_id": "GO:0045944",
  "term_label": "positive regulation of transcription by RNA polymerase II"
}